{
  "gene_symbol": "FAM135A",
  "gene_name": "Protein FAM135A",
  "term_label": "Unknown molecular function",
  "term_id": "UNKNOWN:0001",
  "gene": "UniProtKB:Q9P2D6"
}